{
  "gene_name": "Muscleblind-like protein 3",
  "term_label": "RNA binding",
  "term_id": "GO:0003723",
  "gene": "UniProtKB:Q9NUK0",
  "gene_symbol": "MBNL3"
}